presynaptic membrane organization [GO:0097090] (biological process) Subtypes: GO:0097105 Relationships: is a type of membrane organization [GO:0061024]; is part of synapse organization [GO:0050808] Regulation: regulated by regulation of presynaptic membrane organization [GO:1901629]; negatively regulated by negative regulation of presynaptic membrane organization [GO:1901630]; positively regulated by positive regulation of presynaptic membrane organization [GO:1901631] Also known as: pre-synaptic membrane organization, presynaptic membrane organisation Note: Note that 'presynaptic membrane' in this term should not be mistaken with 'presynaptic active zone'. The latter encompasses more than the former, as it also includes the specialized cortical cytoskeletal matrix in the cell cortex of a presynaptic neuron. References: PMID:19730411 Sources: GOC:BHF, GOC:pr, GOC:sjp Definition: A process which results in the assembly, arrangement of constituent parts, or disassembly of a presynaptic membrane, including any proteins associated with the membrane, but excluding other cellular components. A presynaptic membrane is a specialized area of membrane of the axon terminal that faces the plasma membrane of the neuron or muscle fiber with which the axon terminal establishes a synaptic junction.